{
  "term_label": "cell adhesion molecule binding",
  "gene_symbol": "PCDHB16",
  "gene_name": "Protocadherin beta-16",
  "gene": "UniProtKB:Q9NRJ7",
  "term_id": "GO:0050839"
}